{
  "gene": "UniProtKB:Q8TD84",
  "gene_symbol": "DSCAML1",
  "term_label": "dendrite self-avoidance",
  "term_id": "GO:0070593",
  "gene_name": "Cell adhesion molecule DSCAML1"
}